{
  "term_id": "GO:0005667",
  "term_label": "transcription regulator complex",
  "gene_symbol": "ATF7IP",
  "gene": "UniProtKB:Q6VMQ6",
  "gene_name": "Activating transcription factor 7-interacting protein 1"
}